{
  "gene_name": "Cadherin-12",
  "term_id": "GO:0044331",
  "term_label": "cell-cell adhesion mediated by cadherin",
  "gene": "UniProtKB:P55289",
  "gene_symbol": "CDH12"
}